soluble NSF attachment protein activity [GO:0005483] (molecular function) Also known as: SNAP Relationships: is_a protein-macromolecule adaptor activity [GO:0030674] Definition: Binding to both N-ethylmaleimide-sensitive fusion protein (NSF) and a cis-SNARE complex (i.e. a SNARE complex in which all proteins are associated with the same membrane) and increasing the ATPase activity of NSF, thereby allowing ATP hydrolysis by NSF to disassemble the cis-SNARE complex. References: PMID:14570579, PMID:15556857 Sources: GOC:mah